{
  "gene": "UniProtKB:O75264",
  "term_label": "Unknown cellular component",
  "gene_symbol": "SMIM24",
  "term_id": "UNKNOWN:0003",
  "gene_name": "Small integral membrane protein 24"
}